{
  "gene_name": "Cystic fibrosis transmembrane conductance regulator",
  "gene_symbol": "CFTR",
  "term_label": "chloride transmembrane transport",
  "term_id": "GO:1902476",
  "gene": "UniProtKB:P13569"
}